riboflavin binding [GO:1902444] (molecular function) References: PMID:12083520 Sources: GOC:TermGenie Definition: Binding to riboflavin. Relationships: is a type of GO:0043168; is a type of heterocyclic compound binding [GO:1901363]